{
  "term_id": "UNKNOWN:0003",
  "gene_name": "Keratin-associated protein 5-6",
  "term_label": "Unknown cellular component",
  "gene_symbol": "KRTAP5-6",
  "gene": "UniProtKB:Q6L8G9"
}